{
  "gene_name": "Cytochrome c oxidase subunit 1",
  "term_label": "respiratory chain complex IV",
  "gene": "UniProtKB:P00395",
  "term_id": "GO:0045277",
  "gene_symbol": "MT-CO1"
}